{
  "gene": "UniProtKB:O60683",
  "gene_symbol": "PEX10",
  "term_label": "Unknown molecular function",
  "gene_name": "Peroxisome biogenesis factor 10",
  "term_id": "UNKNOWN:0001"
}